{
  "gene": "UniProtKB:Q8IYJ0",
  "gene_symbol": "PIANP",
  "term_id": "UNKNOWN:0001",
  "term_label": "Unknown molecular function",
  "gene_name": "PILR alpha-associated neural protein"
}